meisosome [GO:0160132] (cellular component) Relationships: is a type of cellular anatomical structure [GO:0110165] References: PMID:36913486 Definition: A cell part that is composed of multifold plasma membrane of the epidermis where it is in direct contact with apical extracellular matrix. Meisosome, or multiple eisome is named because of its superficial similarity to yeast eisosome.